{
  "term_label": "plasma membrane",
  "gene": "UniProtKB:O00499",
  "term_id": "GO:0005886",
  "gene_name": "Myc box-dependent-interacting protein 1",
  "gene_symbol": "BIN1"
}